epigenetic programming in the central cell [GO:0141063] (biological process) Relationships: is a type of genomic imprinting [GO:0071514] References: PMID:28118754 Definition: The establishment of epigenetic modifications (imprints) in a plant central cell, leading to an asymmetry between the two maternal alleles and the paternal allele, and differential expression of the corresponding alleles in the developing endosperm. This can happen through heterochromatin formation or differential chromatin loop formation.